{
  "gene_name": "Protein disulfide-isomerase",
  "gene": "UniProtKB:P07237",
  "term_label": "endoplasmic reticulum",
  "term_id": "GO:0005783",
  "gene_symbol": "P4HB"
}